cell-cell adhesion involved in establishment of planar polarity [GO:0090250] (biological process) Definition: The attachment of one cell to another cell via adhesion molecules that contributes to the establishment of planar cell polarity. Sources: GOC:ascb_2009, GOC:dph, GOC:tb Relationships: is_a cell-cell adhesion [GO:0098609]; is part of GO:0001736